{
  "gene": "UniProtKB:Q16543",
  "gene_name": "Hsp90 co-chaperone Cdc37",
  "gene_symbol": "CDC37",
  "term_label": "protein-folding chaperone binding",
  "term_id": "GO:0051087"
}